mycothiol-dependent formaldehyde dehydrogenase activity [GO:0050607] (molecular function) Also known as: formaldehyde:NAD+ oxidoreductase (mycothiol-formylating), NAD/factor-dependent formaldehyde dehydrogenase activity Definition: Catalysis of the reaction: formaldehyde + mycothiol + NAD+ = S-formylmycothiol + NADH + H+. Relationships: is a type of oxidoreductase activity, acting on the aldehyde or oxo group of donors, NAD or NADP as acceptor [GO:0016620] Sources: EC:1.1.1.306